{
  "term_label": "Unknown cellular component",
  "gene_name": "Putative inactive deoxyuridine 5'-triphosphate nucleotidohydrolase-like protein FLJ16323",
  "gene": "UniProtKB:Q6ZN92",
  "term_id": "UNKNOWN:0003",
  "gene_symbol": "Q6ZN92"
}